{
  "gene_name": "Putative MAGE domain-containing protein MAGEA13P",
  "term_label": "Unknown molecular function",
  "gene": "UniProtKB:A6NCF6",
  "term_id": "UNKNOWN:0001",
  "gene_symbol": "MAGEA13P"
}